mesonephric collecting duct development [GO:0061211] (biological process) Relationships: is a type of collecting duct development [GO:0072044]; is part of mesonephros development [GO:0001823] Definition: The process whose specific outcome is the progression of a collecting duct in the mesonephros over time, from its formation to the mature structure. The collecting duct regulates water, electrolyte and acid-base balance. The collecting duct is the final common path through which urine flows before entering the ureter and then emptying into the bladder. Sources: GOC:mtg_kidney_jan10